{
  "gene": "UniProtKB:A6NFC9",
  "term_label": "olfactory receptor activity",
  "gene_name": "Putative olfactory receptor 2W5 pseudogene",
  "gene_symbol": "OR2W5P",
  "term_id": "GO:0004984"
}